regulation of compound eye cone cell fate specification [GO:0042682] (biological process) Subtypes: negative regulation of compound eye cone cell fate specification [GO:0042683] Sources: GOC:mtg_sensu Relationships: is a type of regulation of cell fate specification [GO:0042659]; RO_0002211 GO:0042679 Definition: Any process that mediates the specification of a cell into a compound eye cone cell.